positive regulation of chemokine (C-C motif) ligand 4 production [GO:0071645] (biological process) Relationships: is a type of GO:0032722; is a type of regulation of chemokine (C-C motif) ligand 4 production [GO:0071643]; RO_0002213 chemokine (C-C motif) ligand 4 production [GO:0071606] Also known as: positive regulation of macrophage inflammatory protein production, positive regulation of CCL4 production, positive regulation of MIP-1b production Definition: Any process that activates or increases the frequency, rate, or extent of production of chemokine (C-C motif) ligand 4. Sources: GOC:mah